CDP-glycerol glycerophosphotransferase activity [GO:0047355] (MF) Also known as: teichoic-acid synthase activity, CDP-glycerol:poly(glycerophosphate) glycerophosphotransferase activity, CDPglycerol glycerophosphotransferase activity, CGPTase activity, cytidine diphosphoglycerol glycerophosphotransferase activity, glycerophosphate synthetase activity, poly(glycerol phosphate) polymerase activity, teichoic acid glycerol transferase activity Sources: EC:2.7.8.12 Relationships: is a type of GO:0016780 Definition: Catalysis of the reaction: glycerophosphate(n) + CDP-glycerol = glycerophosphate(n+1) + CMP.